branchiomeric skeletal muscle development [GO:0014707] (biological process) Relationships: is a type of muscle organ development [GO:0007517]; is a type of skeletal muscle tissue development [GO:0007519] Sources: GOC:mtg_muscle Regulation: regulated by GO:0014711; positively regulated by positive regulation of branchiomeric skeletal muscle development [GO:0014712]; negatively regulated by negative regulation of branchiomeric skeletal muscle development [GO:0014713] Definition: The process whose specific outcome is the progression of the branchiomeric skeletal muscle over time, from its formation to the mature structure. The branchiomeric muscle is derived from cranial mesoderm and controls facial expression, pharyngeal and laryngeal function, operating the jaw. The muscle begins its development with the differentiation of the muscle cells and ends with the mature muscle. Branchiomeric muscles of mammals correspond to the gill musculature of fish.